{
  "gene_symbol": "OLFM1",
  "term_id": "UNKNOWN:0001",
  "term_label": "Unknown molecular function",
  "gene_name": "Noelin",
  "gene": "UniProtKB:Q99784"
}